cellular response to interleukin-1 [GO:0071347] (biological process) Also known as: cellular response to IL-1 Definition: Any process that results in a change in state or activity of a cell (in terms of movement, secretion, enzyme production, gene expression, etc.) as a result of an interleukin-1 stimulus. Relationships: is a type of GO:0070555; is a type of cellular response to cytokine stimulus [GO:0071345] Sources: GOC:mah